{
  "term_id": "GO:0005634",
  "gene": "UniProtKB:Q14587",
  "term_label": "nucleus",
  "gene_name": "Zinc finger protein 268",
  "gene_symbol": "ZNF268"
}